{
  "term_label": "NAD+ poly-ADP-ribosyltransferase activity",
  "gene_name": "GPI-linked NAD(P)(+)--arginine ADP-ribosyltransferase 1",
  "term_id": "GO:0003950",
  "gene": "UniProtKB:P52961",
  "gene_symbol": "ART1"
}